positive regulation of dopamine uptake involved in synaptic transmission [GO:0051586] (biological process) Definition: Any process that activates or increases the frequency, rate or extent of the directed movement of dopamine into a cell. Sources: GOC:ai Also known as: positive regulation of dopamine import involved in synaptic transmission, up regulation of dopamine uptake involved in synaptic transmission, up-regulation of dopamine uptake involved in synaptic transmission, upregulation of dopamine uptake involved in synaptic transmission, activation of dopamine uptake involved in synaptic transmission, stimulation of dopamine uptake involved in synaptic transmission Relationships: is a type of regulation of dopamine uptake involved in synaptic transmission [GO:0051584]; is a type of positive regulation of catecholamine uptake involved in synaptic transmission [GO:0051944]; positively regulates dopamine uptake involved in synaptic transmission [GO:0051583]